{
  "gene": "UniProtKB:P55289",
  "term_id": "GO:0045296",
  "gene_symbol": "CDH12",
  "gene_name": "Cadherin-12",
  "term_label": "cadherin binding"
}